{
  "term_id": "UNKNOWN:0001",
  "term_label": "Unknown molecular function",
  "gene": "UniProtKB:P05452",
  "gene_symbol": "CLEC3B",
  "gene_name": "Tetranectin"
}